{
  "gene": "UniProtKB:O95336",
  "gene_symbol": "PGLS",
  "term_label": "pentose-phosphate shunt, oxidative branch",
  "gene_name": "6-phosphogluconolactonase",
  "term_id": "GO:0009051"
}